'de novo' actin filament nucleation [GO:0070060] (biological process) Also known as: formin-mediated actin filament nucleation, unbranched actin filament nucleation Definition: The actin nucleation process in which actin monomers combine in the absence of any existing actin filaments; elongation of the actin oligomer formed by nucleation leads to the formation of an unbranched filament. References: PMID:17477841 Sources: GOC:mah Relationships: is a type of actin nucleation [GO:0045010]